{
  "gene_name": "Calmodulin-1",
  "term_id": "GO:0005737",
  "term_label": "cytoplasm",
  "gene_symbol": "CALM1",
  "gene": "UniProtKB:P0DP23"
}